{
  "term_label": "signal transduction",
  "gene_name": "TOM1-like protein 1",
  "term_id": "GO:0007165",
  "gene_symbol": "TOM1L1",
  "gene": "UniProtKB:O75674"
}